{
  "term_id": "GO:0005634",
  "gene": "UniProtKB:Q9UIU6",
  "gene_symbol": "SIX4",
  "term_label": "nucleus",
  "gene_name": "Homeobox protein SIX4"
}